{
  "gene": "UniProtKB:Q9UI09",
  "term_id": "UNKNOWN:0001",
  "gene_symbol": "NDUFA12",
  "gene_name": "NADH dehydrogenase [ubiquinone] 1 alpha subcomplex subunit 12",
  "term_label": "Unknown molecular function"
}